{
  "term_id": "GO:0033499",
  "gene_name": "Galactose mutarotase",
  "term_label": "galactose catabolic process via UDP-galactose, Leloir pathway",
  "gene_symbol": "GALM",
  "gene": "UniProtKB:Q96C23"
}